Wnt-Frizzled-LRP5/6 complex assembly [GO:1904701] (biological process) Definition: The aggregation, arrangement and bonding together of a set of components to form a Wnt-Frizzled-LRP5/6 complex. References: PMID:11448771 Sources: GOC:PARL, GOC:TermGenie, GOC:bf, GO_REF:0000079 Also known as: Wnt receptor complex assembly, Wnt-FZD-LRP5/6 trimeric complex assembly, Wnt-FZD-LRP5/6 trimeric complex formation, WNT-FZD-LRP5 complex assembly, WNT-FZD-LRP5 complex formation, WNT-FZD-LRP6 complex assembly, WNT-FZD-LRP6 complex formation, Frizzled-LRP5/6 complex assembly, Frizzled-LRP5/6 complex formation, Wnt-induced Frizzled-LRP5/6 complex assembly, Wnt-induced Frizzled-LRP5/6 complex formation Relationships: is a type of protein-containing complex assembly [GO:0065003] Regulation: regulated by regulation of Wnt-Frizzled-LRP5/6 complex assembly [GO:1904711]; positively regulated by GO:1904712; negatively regulated by negative regulation of Wnt-Frizzled-LRP5/6 complex assembly [GO:1904723]